{
  "gene_name": "Toll-interacting protein",
  "gene_symbol": "TOLLIP",
  "term_label": "ubiquitin binding",
  "gene": "UniProtKB:Q9H0E2",
  "term_id": "GO:0043130"
}